{
  "term_label": "ESCRT I complex",
  "gene_symbol": "VPS37C",
  "term_id": "GO:0000813",
  "gene": "UniProtKB:A5D8V6",
  "gene_name": "Vacuolar protein sorting-associated protein 37C"
}